3',5'-cyclic-AMP phosphodiesterase activity [GO:0004115] (molecular function) Definition: Catalysis of the reaction: 3',5'-cyclic AMP + H2O = AMP + H+. Relationships: is a type of 3',5'-cyclic-nucleotide phosphodiesterase activity [GO:0004114] Subtypes: calmodulin-activated dual specificity 3',5'-cyclic-GMP, 3',5'-cyclic-AMP phosphodiesterase activity [GO:0004117], calmodulin-activated 3',5'-cyclic-AMP phosphodiesterase activity [GO:0140761] Sources: GOC:ai, RHEA:25277 Also known as: 3',5' cAMP-specific phosphodiesterase activity, 3',5'-cAMP-specific phosphodiesterase activity, 3',5'-cyclic-AMP-specific phosphodiesterase activity, adenosine 3',5'-cyclophosphate-specific phosphodiesterase activity, cAMP-specific phosphodiesterase activity, cyclic AMP-specific phosphodiesterase activity